{
  "term_id": "GO:0044458",
  "gene": "UniProtKB:D6RGH6",
  "gene_symbol": "MCIDAS",
  "term_label": "motile cilium assembly",
  "gene_name": "Multicilin"
}